C-C motif chemokine 21 receptor activity [GO:0038121] (molecular function) Relationships: is a type of C-C chemokine receptor activity [GO:0016493]; is part of chemokine (C-C motif) ligand 21 signaling pathway [GO:0038116]; has part GO:0035758 Also known as: CCL21 receptor activity Definition: Combining with the C-C motif chemokine 21 (CCL21) and transmitting the signal from one side of the membrane to the other to initiate a change in cell activity. References: PMID:15059845 Sources: GOC:signaling